{
  "term_label": "Unknown cellular component",
  "gene_symbol": "CFAP73",
  "gene_name": "Cilia- and flagella-associated protein 73",
  "gene": "UniProtKB:A6NFT4",
  "term_id": "UNKNOWN:0003"
}